rhombomere 4 development [GO:0021570] (BP) Definition: The process whose specific outcome is the progression of rhombomere 4 over time, from its formation to the mature structure. Rhombomeres are transverse segments of the developing rhombencephalon. Rhombomeres are lineage restricted, express different genes from one another, and adopt different developmental fates. Rhombomeres are numbered in anterior to posterior order. Sources: GOC:cls, GOC:curators, GOC:dgh, GOC:dph, GOC:jid Relationships: is a type of rhombomere development [GO:0021546]